regulation of transcriptional start site selection at RNA polymerase II promoter [GO:0001178] (biological process) Sources: GOC:txnOH Definition: Any process that modulates the rate, frequency or extent of a process involved in the selection of the specific location within the template strand of an RNA polymerase II promoter for hybridization of the cognate ribonucleotides and formation of first phosphodiester bond within the nascent transcript. Relationships: is a type of regulation of transcription, start site selection [GO:0010630]; is a type of regulation of transcription initiation by RNA polymerase II [GO:0060260]; RO_0002211 GO:0001174 Also known as: regulation of transcription start site selection at RNA polymerase II promoter